tRNA methylation [GO:0030488] (biological process) Sources: GOC:mah Definition: The posttranscriptional addition of methyl groups to specific residues in a tRNA molecule. Regulation: regulated by regulation of tRNA methylation [GO:0110002]; positively regulated by positive regulation of tRNA methylation [GO:0110004] Subtypes: tRNA nucleoside ribose methylation [GO:0002128], GO:0002939, tRNA N2-guanine methylation [GO:0002940], tRNA m2,2-guanine biosynthesis [GO:0002942], tRNA C5-cytosine methylation [GO:0002946], mitochondrial tRNA methylation [GO:0070901], 5-carbamoylmethyl uridine residue modification [GO:0080178], tRNA (guanine-N7)-methylation [GO:0106004], GO:0106217 Relationships: is a type of GO:0001510; is a type of tRNA modification [GO:0006400]